{
  "term_id": "UNKNOWN:0002",
  "gene_symbol": "TKTL2",
  "term_label": "Unknown biological process",
  "gene_name": "Transketolase-like protein 2",
  "gene": "UniProtKB:Q9H0I9"
}